{
  "gene_name": "Ras-related protein Rab-11A",
  "gene_symbol": "RAB11A",
  "gene": "UniProtKB:P62491",
  "term_id": "GO:0005794",
  "term_label": "Golgi apparatus"
}